aerobactin biosynthetic process [GO:0019270] (biological process) Definition: The chemical reactions and pathways resulting in the formation of aerobactin (C22H36N4O13), a hydroxamate iron transport compound. It is a conjugate of 6-(N-acetyl-N-hydroxylamine)-2-aminohexanoic acid and citric acid. Sources: GOC:ai Relationships: is a type of modified amino acid biosynthetic process [GO:0042398]; is a type of tricarboxylic acid biosynthetic process [GO:0072351] Also known as: aerobactin anabolism, aerobactin biosynthesis, aerobactin formation, aerobactin synthesis